regulation of metaphase/anaphase transition of cell cycle [GO:1902099] (biological process) Sources: GOC:TermGenie, GOC:mtg_cell_cycle Definition: Any process that modulates the frequency, rate or extent of metaphase/anaphase transition of cell cycle. Relationships: is a type of regulation of sister chromatid segregation [GO:0033045]; is a type of regulation of cell cycle phase transition [GO:1901987]; regulates GO:0044784 Subtypes: regulation of mitotic metaphase/anaphase transition [GO:0030071], negative regulation of metaphase/anaphase transition of cell cycle [GO:1902100], positive regulation of metaphase/anaphase transition of cell cycle [GO:1902101], regulation of metaphase/anaphase transition of meiotic cell cycle [GO:1902102]